{
  "gene_symbol": "FCGBP",
  "gene_name": "IgGFc-binding protein",
  "term_id": "UNKNOWN:0002",
  "term_label": "Unknown biological process",
  "gene": "UniProtKB:Q9Y6R7"
}